cellular response to interleukin-12 [GO:0071349] (biological process) Definition: Any process that results in a change in state or activity of a cell (in terms of movement, secretion, enzyme production, gene expression, etc.) as a result of an interleukin-12 stimulus. Sources: GOC:mah Also known as: cellular response to IL-12 Relationships: is_a response to interleukin-12 [GO:0070671]; is a type of GO:0071345